glutathionylspermidine amidase activity [GO:0008884] (molecular function) Sources: EC:3.5.1.78 Also known as: GSP amidase activity, gamma-L-glutamyl-L-cysteinyl-glycine:spermidine amidase activity, glutathionylspermidine amidohydrolase (spermidine-forming) activity Definition: Catalysis of the reaction: N1-(gamma-L-glutamyl-L-cysteinyl-glycyl)-spermidine + H2O = gamma-L-glutamyl-L-cysteinyl-glycine + spermidine. Relationships: is a type of hydrolase activity, acting on carbon-nitrogen (but not peptide) bonds, in linear amides [GO:0016811]